N-sulfoglucosamine-3-sulfatase activity [GO:0033889] (molecular function) Sources: EC:3.1.6.15 Definition: Catalysis of the hydrolysis of the 3-sulfate groups of the N-sulfo-D-glucosamine 3-O-sulfate units of heparin. Also known as: chondroitinsulfatase activity, N-sulfo-3-sulfoglucosamine 3-sulfohydrolase activity Relationships: is a type of GO:0008484